{
  "gene_symbol": "BACH1",
  "term_id": "GO:0000981",
  "term_label": "DNA-binding transcription factor activity, RNA polymerase II-specific",
  "gene_name": "Transcription regulator protein BACH1",
  "gene": "UniProtKB:O14867"
}